ESC/E(Z) complex [GO:0035098] (cellular component) Also known as: Extra Sex Combs/Enhancer of Zeste complex, PRC2 complex, polycomb repressive complex 2 Relationships: is a type of PcG protein complex [GO:0031519]; is a type of histone methyltransferase complex [GO:0035097] References: PMID:12408863, PMID:12408864, PMID:17107999, PMID:20064375, PMID:31123059, PMID:33232890 Sources: GOC:bf, GOC:krc, GOC:sp Definition: A multimeric protein complex that can methylate lysine-27 and lysine-9 residues of histone H3. In Drosophila the core subunits of the complex include ESC, E(Z), CAF1 (NURF-55) and SU(Z)12. In mammals the core subunits of the complex include EED, EZH2, SUZ12 and RBBP4.